{
  "term_id": "UNKNOWN:0001",
  "gene": "UniProtKB:Q8NAV1",
  "term_label": "Unknown molecular function",
  "gene_symbol": "PRPF38A",
  "gene_name": "Pre-mRNA-splicing factor 38A"
}